{
  "term_label": "actin filament",
  "term_id": "GO:0005884",
  "gene_name": "Protein diaphanous homolog 1",
  "gene": "UniProtKB:O60610",
  "gene_symbol": "DIAPH1"
}